positive regulation of conjugation with cellular fusion [GO:0031139] (biological process) Subtypes: induction of conjugation with cellular fusion [GO:0010514], signal transduction involved in positive regulation of conjugation with cellular fusion [GO:0032005], positive regulation of signal transduction involved in conjugation with cellular fusion [GO:0060239], GO:0071631, positive regulation of induction of conjugation with cellular fusion [GO:1900237] Sources: GOC:mah Also known as: up regulation of conjugation with cellular fusion, up-regulation of conjugation with cellular fusion, upregulation of conjugation with cellular fusion, activation of conjugation with cellular fusion, stimulation of conjugation with cellular fusion Relationships: is a type of regulation of conjugation with cellular fusion [GO:0031137]; is a type of positive regulation of reproductive process [GO:2000243]; positively regulates conjugation with cellular fusion [GO:0000747] Definition: Any process that increases the rate or frequency of conjugation with cellular fusion.